{
  "gene": "UniProtKB:Q709F0",
  "gene_name": "Acyl-CoA dehydrogenase family member 11",
  "gene_symbol": "ACAD11",
  "term_label": "cytoplasm",
  "term_id": "GO:0005737"
}